{
  "term_id": "GO:0038158",
  "gene": "UniProtKB:O00165",
  "term_label": "granulocyte colony-stimulating factor signaling pathway",
  "gene_name": "HCLS1-associated protein X-1",
  "gene_symbol": "HAX1"
}